{
  "gene": "UniProtKB:Q96I25",
  "gene_symbol": "RBM17",
  "term_id": "GO:0000380",
  "term_label": "alternative mRNA splicing, via spliceosome",
  "gene_name": "Splicing factor 45"
}